{
  "gene_symbol": "CCNI",
  "term_label": "cyclin-dependent protein kinase holoenzyme complex",
  "gene_name": "Cyclin-I",
  "gene": "UniProtKB:Q14094",
  "term_id": "GO:0000307"
}